{
  "gene_name": "Eukaryotic translation initiation factor 3 subunit L",
  "term_id": "GO:0006413",
  "term_label": "translational initiation",
  "gene": "UniProtKB:Q9Y262",
  "gene_symbol": "EIF3L"
}